{
  "term_id": "GO:0005783",
  "gene_symbol": "KLHL14",
  "gene": "UniProtKB:Q9P2G3",
  "term_label": "endoplasmic reticulum",
  "gene_name": "Kelch-like protein 14"
}